intronic transcription regulatory region sequence-specific DNA binding [GO:0001161] (molecular function) Sources: GOC:txnOH Note: To minimize ambiguity in the use of the word "promoter" in GO, we have chosen the phrase "transcription regulatory region" to refer to all of the regulatory regions. Regulatory regions in the DNA which control initiation may include the "core promoter" where the basal transcription machinery binds, the "core promoter proximal region" where regulatory factors other than the basal machinery bind. There are also additional regulatory regions, in both the DNA and the RNA transcript, which regulate elongation or termination of transcription. Also known as: intronic transcription regulatory region DNA binding Subtypes: RNA polymerase II intronic transcription regulatory region sequence-specific DNA binding [GO:0001162] Definition: Binding to an intronic DNA sequence that regulates the transcription of the transcript it is contained within. Relationships: is a type of transcription cis-regulatory region binding [GO:0000976]